{
  "gene_symbol": "NKX6-1",
  "term_id": "GO:0000981",
  "term_label": "DNA-binding transcription factor activity, RNA polymerase II-specific",
  "gene_name": "Homeobox protein Nkx-6.1",
  "gene": "UniProtKB:P78426"
}